ATPase complex [GO:1904949] (cellular component) Note: An example of this is VPS4 in Saccharomyces cerevisiae (UniProt ID P52917) in PMID:9606181 (inferred from direct assay). Relationships: is_a catalytic complex [GO:1902494] Subtypes: proton-transporting V-type ATPase complex [GO:0033176], GO:0062091, SWI/SNF superfamily-type complex [GO:0070603], cytosolic [4Fe-4S] assembly scaffold complex [GO:1904564], archaeal proton-transporting A-type ATPase complex [GO:1990490], ESCRT IV complex [GO:1990621] Also known as: VPS4 complex References: PMID:9606181 Sources: GOC:TermGenie, GOC:bhm, GO_REF:0000088 Definition: A protein complex which is capable of ATPase activity.